{
  "gene_symbol": "JADE1",
  "gene_name": "Protein Jade-1",
  "term_id": "GO:0000123",
  "gene": "UniProtKB:Q6IE81",
  "term_label": "histone acetyltransferase complex"
}